{
  "gene": "UniProtKB:Q16445",
  "term_label": "GABA-gated chloride ion channel activity",
  "gene_symbol": "GABRA6",
  "gene_name": "Gamma-aminobutyric acid receptor subunit alpha-6",
  "term_id": "GO:0022851"
}